asymmetric Golgi ribbon formation [GO:0090164] (biological process) Subtypes: GO:0090165 Relationships: is a type of Golgi ribbon formation [GO:0090161]; is part of establishment of epithelial cell polarity [GO:0090162] Definition: The asymmetric formation of a continuous ribbon of interconnected Golgi stacks of flat cisternae that contributes to the establishment of epithelial cell polarity. Sources: GOC:ascb_2009, GOC:dph, GOC:tb